{
  "term_label": "cytosolic large ribosomal subunit",
  "gene": "UniProtKB:P84098",
  "gene_symbol": "RPL19",
  "gene_name": "Large ribosomal subunit protein eL19",
  "term_id": "GO:0022625"
}